{
  "term_label": "Z disc",
  "gene_name": "Synaptopodin",
  "gene": "UniProtKB:Q8N3V7",
  "gene_symbol": "SYNPO",
  "term_id": "GO:0030018"
}